{
  "term_id": "GO:0007026",
  "gene_symbol": "BMERB1",
  "term_label": "negative regulation of microtubule depolymerization",
  "gene_name": "bMERB domain-containing protein 1",
  "gene": "UniProtKB:Q96MC5"
}